positive regulation of cardiac muscle contraction [GO:0060452] (biological process) Definition: Any process that increases the frequency, rate or extent of cardiac muscle contraction. Relationships: is a type of positive regulation of heart contraction [GO:0045823]; is a type of positive regulation of striated muscle contraction [GO:0045989]; is a type of regulation of cardiac muscle contraction [GO:0055117]; positively regulates cardiac muscle contraction [GO:0060048] Sources: GOC:dph, GOC:tb